regulation of triglyceride transport [GO:1905883] (biological process) Subtypes: negative regulation of triglyceride transport [GO:1905884], GO:1905885 Also known as: regulation of triacylglycerol transport Definition: Any process that modulates the frequency, rate or extent of triglyceride transport. Relationships: is a type of regulation of acylglycerol transport [GO:1901506]; regulates triglyceride transport [GO:0034197] References: PMID:25849533 Sources: GOC:TermGenie, GO_REF:0000058